{
  "gene_name": "Humanin-like 7",
  "gene_symbol": "MTRNR2L7",
  "gene": "UniProtKB:P0CJ74",
  "term_label": "receptor antagonist activity",
  "term_id": "GO:0048019"
}